alpha-2B adrenergic receptor binding [GO:0031695] (molecular function) Sources: GOC:mah, GOC:nln Relationships: is a type of adrenergic receptor binding [GO:0031690] Also known as: alpha-2B adrenergic receptor ligand Definition: Binding to an alpha-2B adrenergic receptor.